URM1 transferase activity [GO:0042294] (molecular function) Relationships: is_a ubiquitin-like protein transferase activity [GO:0019787] Definition: Catalysis of the transfer of URM1 from one protein to another via the reaction X-URM1 + Y = Y-URM1 + X, where both X-URM1 and Y-URM1 are covalent linkages. Subtypes: URM1 conjugating enzyme activity [GO:0061658], URM1 ligase activity [GO:0061667] References: PMID:12826404 Sources: GOC:mah